glucan 1,4-beta-glucosidase activity [GO:0031217] (molecular function) Relationships: is a type of beta-glucosidase activity [GO:0008422] Sources: EC:3.2.1.74, GOC:mlg Definition: Catalysis of the hydrolysis of (1->4) linkages in (1->4)-beta-D-glucans, to remove successive glucose units. Also known as: 1,4-beta-D-glucan glucohydrolase activity, beta-1,4-beta-glucanase activity, beta-1,4-glucanase activity, exo-1,4-beta-glucanase activity, exo-1,4-beta-glucosidase activity, exo-beta-1,4-glucanase activity, exo-beta-1,4-glucosidase activity, exocellulase activity, exo-1,4-beta-D-glucosidase activity